{
  "gene_symbol": "ACADVL",
  "gene_name": "Very long-chain specific acyl-CoA dehydrogenase, mitochondrial",
  "term_id": "UNKNOWN:0003",
  "gene": "UniProtKB:P49748",
  "term_label": "Unknown cellular component"
}